{
  "term_id": "UNKNOWN:0002",
  "gene": "UniProtKB:Q9NQ92",
  "term_label": "Unknown biological process",
  "gene_name": "Coordinator of PRMT5 and differentiation stimulator",
  "gene_symbol": "COPRS"
}